(+)-delta-cadinene-8-hydroxylase activity [GO:0102947] (MF) Relationships: is a type of GO:0016709 Sources: GOC:pz Definition: Catalysis of the reaction: H+ + (+)-delta-cadinene + NADPH + O2 = 8-hydroxy-(+)-delta-cadinene + NADP + H2O.